{
  "gene": "UniProtKB:O76093",
  "gene_name": "Fibroblast growth factor 18",
  "term_label": "type 2 fibroblast growth factor receptor binding",
  "term_id": "GO:0005111",
  "gene_symbol": "FGF18"
}